negative regulation of fibroblast growth factor receptor signaling pathway [GO:0040037] (biological process) Definition: Any process that stops, prevents, or reduces the frequency, rate or extent of fibroblast growth factor receptor signaling pathway activity. Also known as: down regulation of fibroblast growth factor receptor signaling pathway, down-regulation of fibroblast growth factor receptor signaling pathway, downregulation of fibroblast growth factor receptor signaling pathway, negative regulation of FGF receptor signaling pathway, negative regulation of FGF receptor signalling pathway, negative regulation of FGFR signaling pathway, inhibition of fibroblast growth factor receptor signaling pathway Subtypes: negative regulation of fibroblast growth factor receptor signaling pathway involved in neural plate anterior/posterior pattern formation [GO:2000314], GO:2000703 Relationships: is a type of negative regulation of signal transduction [GO:0009968]; is a type of regulation of fibroblast growth factor receptor signaling pathway [GO:0040036]; is a type of negative regulation of cellular response to growth factor stimulus [GO:0090288]; negatively regulates GO:0008543 Sources: GOC:go_curators